{
  "term_id": "GO:0005929",
  "term_label": "cilium",
  "gene": "UniProtKB:Q9Y547",
  "gene_name": "Intraflagellar transport protein 25 homolog",
  "gene_symbol": "IFT25"
}